{
  "gene_name": "D(3) dopamine receptor",
  "gene_symbol": "DRD3",
  "term_label": "G protein-coupled receptor activity",
  "term_id": "GO:0004930",
  "gene": "UniProtKB:P35462"
}